positive regulation of fever generation by positive regulation of prostaglandin biosynthesis [GO:0071811] (biological process) Sources: GOC:BHF, GOC:dph, GOC:mah Relationships: is a type of positive regulation of prostaglandin biosynthetic process [GO:0031394]; is a type of positive regulation of fever generation [GO:0031622] Definition: Any process that increases the rate or extent of fever generation via positive regulation of the frequency, rate or extent of the chemical reactions and pathways resulting in the formation of prostaglandin.